mitotic DNA replication preinitiation complex assembly [GO:1902977] (biological process) Sources: GOC:TermGenie, GO_REF:0000060 Relationships: is a type of DNA replication preinitiation complex assembly [GO:0071163]; is_a mitotic cell cycle process [GO:1903047]; is part of mitotic DNA replication [GO:1902969] Definition: Any DNA replication preinitiation complex assembly that is involved in mitotic cell cycle. Also known as: DNA replication preinitiation complex formation involved in mitotic cell cycle, pre-IC complex assembly involved in mitotic cell cycle